{
  "gene_symbol": "SSR4",
  "gene": "UniProtKB:P51571",
  "term_id": "GO:0012505",
  "gene_name": "Translocon-associated protein subunit delta",
  "term_label": "endomembrane system"
}